{
  "term_id": "GO:0006511",
  "term_label": "ubiquitin-dependent protein catabolic process",
  "gene_name": "E3 ubiquitin-protein ligase RNF125",
  "gene_symbol": "RNF125",
  "gene": "UniProtKB:Q96EQ8"
}